{
  "term_id": "GO:0004879",
  "gene_symbol": "NR1I2",
  "gene_name": "Nuclear receptor subfamily 1 group I member 2",
  "gene": "UniProtKB:O75469",
  "term_label": "nuclear receptor activity"
}